phospholipid transfer activity [GO:0120014] (molecular function) Definition: Removes a phospholipid from a membrane or a monolayer lipid particle, transports it through the aqueous phase while protected in a hydrophobic pocket, and brings it to an acceptor membrane or lipid particle. Subtypes: phosphatidylinositol transfer activity [GO:0008526], phosphatidylcholine transfer activity [GO:0120019], GO:0140338, phosphatidylglycerol transfer activity [GO:0140339], phosphatidylserine transfer activity [GO:0140343], ceramide 1-phosphate transfer activity [GO:1902388], GO:1904121, GO:1990050 Also known as: phospholipid carrier activity, intermembrane phospholipid transfer activity Relationships: is a type of phospholipid transporter activity [GO:0005548]; is a type of GO:0120013; has part GO:0005543 References: PMID:20823909, PMID:24220498, PMID:25797198 Sources: GOC:krc